{
  "gene_name": "Stathmin-4",
  "term_id": "GO:0015631",
  "gene": "UniProtKB:Q9H169",
  "gene_symbol": "STMN4",
  "term_label": "tubulin binding"
}